sodium ion uniporter activity [GO:0022818] (molecular function) Sources: GOC:mtg_transport, ISBN:0815340729 Definition: Catalysis of the active transport of a sodium ion across a membrane by a mechanism involving conformational change, where energy for active transport is derived from membrane potential if the solute is charged. Relationships: is_a sodium ion transmembrane transporter activity [GO:0015081]; is a type of membrane potential driven uniporter activity [GO:0022810]